negative regulation of synapse maturation [GO:2000297] (BP) Definition: Any process that stops, prevents or reduces the frequency, rate or extent of synapse maturation. Sources: GOC:mah Also known as: negative regulation of synaptic maturation Relationships: is a type of negative regulation of developmental process [GO:0051093]; is a type of GO:0090128; is a type of negative regulation of synapse organization [GO:1905809]; negatively regulates synapse maturation [GO:0060074]